{
  "term_id": "UNKNOWN:0002",
  "gene_name": "Fanconi anemia group E protein",
  "gene_symbol": "FANCE",
  "gene": "UniProtKB:Q9HB96",
  "term_label": "Unknown biological process"
}